response to perphenazine [GO:0097334] (biological process) Definition: Any process that results in a change in state or activity of a cell or an organism (in terms of movement, secretion, enzyme production, gene expression, etc.) as a result of a perphenazine stimulus. Perphenazine is a phenothiazine derivative having a chloro substituent at the 2-position and a 3-[4-(2-hydroxyethyl)piperazin-1-yl]propyl group at the N-10 position. Sources: GOC:pr Relationships: is a type of response to alcohol [GO:0097305]; is a type of response to nitrogen compound [GO:1901698]